{
  "term_label": "cytoplasmic microtubule",
  "term_id": "GO:0005881",
  "gene_name": "UPF0602 protein C4orf47",
  "gene": "UniProtKB:A7E2U8",
  "gene_symbol": "C4orf47"
}